{
  "term_label": "cell adhesion molecule binding",
  "gene_symbol": "PCDH7",
  "term_id": "GO:0050839",
  "gene_name": "Protocadherin-7",
  "gene": "UniProtKB:O60245"
}